{
  "gene": "UniProtKB:P0CL80",
  "term_id": "UNKNOWN:0003",
  "gene_symbol": "GAGE12F",
  "term_label": "Unknown cellular component",
  "gene_name": "G antigen 12F"
}